{
  "gene_symbol": "OR6B2",
  "gene_name": "Olfactory receptor 6B2",
  "term_id": "UNKNOWN:0002",
  "gene": "UniProtKB:Q6IFH4",
  "term_label": "Unknown biological process"
}